{
  "gene": "UniProtKB:Q9P0K7",
  "gene_symbol": "RAI14",
  "term_label": "Unknown biological process",
  "gene_name": "Ankycorbin",
  "term_id": "UNKNOWN:0002"
}